{
  "gene": "UniProtKB:A0A7P0T9M0",
  "gene_name": "Uncharacterized protein",
  "gene_symbol": "A0A7P0T9M0",
  "term_label": "Unknown cellular component",
  "term_id": "UNKNOWN:0003"
}